{
  "term_id": "UNKNOWN:0001",
  "gene": "UniProtKB:Q9NXE8",
  "gene_symbol": "CWC25",
  "term_label": "Unknown molecular function",
  "gene_name": "Pre-mRNA-splicing factor CWC25 homolog"
}